{
  "term_id": "GO:0016538",
  "gene": "UniProtKB:P41002",
  "gene_symbol": "CCNF",
  "gene_name": "Cyclin-F",
  "term_label": "cyclin-dependent protein serine/threonine kinase regulator activity"
}